Cul4-RING E3 ubiquitin ligase complex [GO:0080008] (cellular component) Definition: A ubiquitin ligase complex in which a cullin from the Cul4 family and a RING domain protein form the catalytic core; substrate specificity is conferred by an adaptor protein. Relationships: is a type of cullin-RING ubiquitin ligase complex [GO:0031461] References: PMID:16792691, PMID:18223036, PMID:18552200 Subtypes: GO:0031464, Cul4B-RING E3 ubiquitin ligase complex [GO:0031465], CLRC complex [GO:0043494]